{
  "gene_name": "Adhesion G protein-coupled receptor A2",
  "term_label": "central nervous system development",
  "term_id": "GO:0007417",
  "gene_symbol": "ADGRA2",
  "gene": "UniProtKB:Q96PE1"
}